{
  "gene": "UniProtKB:P49407",
  "gene_symbol": "ARRB1",
  "term_label": "positive regulation of ERK1 and ERK2 cascade",
  "gene_name": "Beta-arrestin-1",
  "term_id": "GO:0070374"
}